positive regulation of collagen catabolic process [GO:0120158] (biological process) Sources: GOC:dph, GOC:tb Also known as: positive regulation of collagen breakdown, positive regulation of collagen catabolism, positive regulation of collagen degradation, up regulation of collagen catabolic process, up-regulation of collagen catabolic process, upregulation of collagen catabolic process, activation of collagen catabolic process Definition: Any process that activates or increases the frequency, rate or extent of collagen catabolism. Collagen catabolism is the proteolytic chemical reactions and pathways resulting in the breakdown of collagen in the extracellular matrix. Relationships: is a type of positive regulation of catabolic process [GO:0009896]; is a type of regulation of collagen catabolic process [GO:0010710]; is a type of positive regulation of collagen metabolic process [GO:0010714]; positively regulates collagen catabolic process [GO:0030574]